{
  "term_id": "GO:0005886",
  "gene_symbol": "ASAP1",
  "gene_name": "Arf-GAP with SH3 domain, ANK repeat and PH domain-containing protein 1",
  "term_label": "plasma membrane",
  "gene": "UniProtKB:Q9ULH1"
}